{
  "term_label": "Unknown molecular function",
  "gene": "UniProtKB:Q9BXW3",
  "term_id": "UNKNOWN:0001",
  "gene_symbol": "SNHG12",
  "gene_name": "Putative uncharacterized protein SNHG12"
}